{
  "gene_symbol": "SLAMF7",
  "gene_name": "SLAM family member 7",
  "term_id": "GO:0009897",
  "term_label": "external side of plasma membrane",
  "gene": "UniProtKB:Q9NQ25"
}